{
  "gene_symbol": "MIPEP",
  "gene_name": "Mitochondrial intermediate peptidase",
  "term_label": "metalloendopeptidase activity",
  "term_id": "GO:0004222",
  "gene": "UniProtKB:Q99797"
}